1,4-dichlorobenzene catabolic process [GO:0019261] (biological process) References: PMID:9148781 Sources: GOC:ai Relationships: is a type of GO:0009056; is a type of benzene-containing compound metabolic process [GO:0042537]; is a type of organohalogen metabolic process [GO:0090345] Definition: The chemical reactions and pathways resulting in the breakdown of 1,4-dichlorobenzene (p-dichlorobenzene or paramoth), a derivative of benzene with two chlorine atoms attached at opposite positions on the ring. Also known as: 1,4-dichlorobenzene breakdown, 1,4-dichlorobenzene catabolism, 1,4-dichlorobenzene degradation